{
  "gene_name": "Homeobox protein Hox-B7",
  "term_id": "GO:0006357",
  "gene": "UniProtKB:P09629",
  "term_label": "regulation of transcription by RNA polymerase II",
  "gene_symbol": "HOXB7"
}